{
  "term_id": "GO:0031530",
  "gene": "UniProtKB:O43555",
  "term_label": "gonadotropin-releasing hormone receptor binding",
  "gene_symbol": "GNRH2",
  "gene_name": "Progonadoliberin-2"
}